{
  "gene_symbol": "FNDC3A",
  "term_id": "GO:0005737",
  "gene": "UniProtKB:Q9Y2H6",
  "gene_name": "Fibronectin type-III domain-containing protein 3A",
  "term_label": "cytoplasm"
}